{
  "gene": "UniProtKB:Q8N4Q0",
  "term_label": "Unknown biological process",
  "gene_symbol": "PTGR3",
  "gene_name": "Prostaglandin reductase 3",
  "term_id": "UNKNOWN:0002"
}